{
  "gene_name": "Nuclear RNA export factor 3",
  "term_label": "nucleus",
  "gene_symbol": "NXF3",
  "gene": "UniProtKB:Q9H4D5",
  "term_id": "GO:0005634"
}